fructose-2,6-bisphosphate 2-phosphatase activity [GO:0004331] (molecular function) Sources: EC:3.1.3.46 Relationships: is a type of sugar-phosphatase activity [GO:0050308] Definition: Catalysis of the reaction: D-fructose 2,6-bisphosphate + H2O = D-fructose-6-phosphate + phosphate. Also known as: D-fructose-2,6-bisphosphate 2-phosphohydrolase activity, beta-D-fructose-2,6-bisphosphate 2-phosphohydrolase activity, fructose-2,6-bisphosphatase activity